{
  "gene": "UniProtKB:Q5S007",
  "gene_symbol": "LRRK2",
  "gene_name": "Leucine-rich repeat serine_threonine-protein kinase 2",
  "term_id": "GO:0031344",
  "term_label": "regulation of cell projection organization"
}